mitochondrion transport along microtubule [GO:0047497] (biological process) Also known as: mitochondrial migration along microtubule, mitochondrial transport along microtubule Sources: GOC:ecd Subtypes: axonal transport of mitochondrion [GO:0019896], dendritic transport of mitochondrion [GO:0098939] Relationships: is a type of GO:0034643; is a type of organelle transport along microtubule [GO:0072384] Definition: The directed movement of a mitochondrion along a microtubule, mediated by motor proteins.